{
  "term_label": "cholesterol biosynthetic process",
  "gene_name": "Mevalonate kinase",
  "gene": "UniProtKB:Q03426",
  "gene_symbol": "MVK",
  "term_id": "GO:0006695"
}